{
  "term_label": "actin cytoskeleton organization",
  "term_id": "GO:0030036",
  "gene_symbol": "SMTNL2",
  "gene_name": "Smoothelin-like protein 2",
  "gene": "UniProtKB:Q2TAL5"
}